mitochondrial large ribosomal subunit [GO:0005762] (cellular component) Definition: The larger of the two subunits of a mitochondrial ribosome. Two sites on the ribosomal large subunit are involved in translation: the aminoacyl site (A site) and peptidyl site (P site). Sources: GOC:mcc Also known as: 39S ribosomal subunit, mitochondrial Relationships: is a type of organellar large ribosomal subunit [GO:0000315]; is a type of mitochondrial protein-containing complex [GO:0098798]; BFO_0000050 mitochondrial ribosome [GO:0005761]